{
  "gene_symbol": "CCN6",
  "gene_name": "Cellular communication network factor 6",
  "term_id": "GO:0005178",
  "term_label": "integrin binding",
  "gene": "UniProtKB:O95389"
}